{
  "term_id": "UNKNOWN:0001",
  "gene_symbol": "LINC00301",
  "gene": "UniProtKB:Q8NCQ3",
  "gene_name": "Putative uncharacterized protein encoded by LINC00301",
  "term_label": "Unknown molecular function"
}